protein succinylation [GO:0018335] (biological process) Also known as: protein amino acid succinylation Sources: GOC:bf Relationships: is a type of GO:0043543 Definition: The modification of a protein by the addition of a succinyl group (CO-CH2-CH2-CO) to an amino acid residue.